{
  "gene_name": "Putative nuclease HARBI1",
  "term_id": "UNKNOWN:0001",
  "gene_symbol": "HARBI1",
  "gene": "UniProtKB:Q96MB7",
  "term_label": "Unknown molecular function"
}